phosphatidylinositol 3-kinase complex, class III [GO:0035032] (cellular component) References: PMID:9255069 Sources: GOC:bf Subtypes: phosphatidylinositol 3-kinase complex, class III, type I [GO:0034271], phosphatidylinositol 3-kinase complex, class III, type II [GO:0034272] Also known as: class III PI3K complex, phosphoinositide 3-kinase complex, class III Relationships: is a type of phosphatidylinositol 3-kinase complex [GO:0005942] Definition: A phosphatidylinositol 3-kinase complex that contains a catalytic class III phosphoinositide 3-kinase (PI3K) subunit bound to a regulatory (adaptor) subunit. Additional adaptor proteins may be present. Class III PI3Ks have a substrate specificity restricted to phosphatidylinositol (PI).